{
  "gene_name": "Putative solute carrier organic anion transporter family member 1B7",
  "term_id": "GO:0043252",
  "gene": "UniProtKB:G3V0H7",
  "term_label": "sodium-independent organic anion transport",
  "gene_symbol": "SLCO1B7"
}